{
  "gene_name": "Zinc finger protein 69 homolog B",
  "gene": "UniProtKB:Q9UJL9",
  "term_label": "regulation of transcription by RNA polymerase II",
  "gene_symbol": "ZFP69B",
  "term_id": "GO:0006357"
}